{
  "term_id": "GO:0048168",
  "gene": "UniProtKB:Q7LC44",
  "gene_name": "Activity-regulated cytoskeleton-associated protein",
  "gene_symbol": "ARC",
  "term_label": "regulation of neuronal synaptic plasticity"
}